{
  "gene_symbol": "PSMD14",
  "gene": "UniProtKB:O00487",
  "gene_name": "26S proteasome non-ATPase regulatory subunit 14",
  "term_id": "GO:0043161",
  "term_label": "proteasome-mediated ubiquitin-dependent protein catabolic process"
}